{
  "gene_name": "RWD domain-containing protein 2A",
  "term_label": "Unknown cellular component",
  "gene_symbol": "RWDD2A",
  "gene": "UniProtKB:Q9UIY3",
  "term_id": "UNKNOWN:0003"
}